{
  "gene_symbol": "SLC9A1",
  "term_label": "sodium ion import across plasma membrane",
  "term_id": "GO:0098719",
  "gene": "UniProtKB:P19634",
  "gene_name": "Sodium_hydrogen exchanger 1"
}